{
  "gene_name": "Serine hydrolase-like protein",
  "gene_symbol": "SERHL",
  "term_label": "Unknown cellular component",
  "gene": "UniProtKB:Q9NQF3",
  "term_id": "UNKNOWN:0003"
}